regulation of endoribonuclease activity [GO:0060699] (biological process) Definition: Any process that modulates the rate, frequency or extent of the catalysis of the hydrolysis of ester linkages within ribonucleic acid by creating internal breaks. Relationships: is a type of regulation of ribonuclease activity [GO:0060700]; regulates RNA endonuclease activity [GO:0004521] Sources: GOC:dph, GOC:tb Subtypes: negative regulation of endoribonuclease activity [GO:0060702]